positive regulation of chemokine (C-C motif) ligand 20 production [GO:1903886] (biological process) Also known as: positive regulation of C-C motif chemokine 20 production, positive regulation of CCL-20 production, positive regulation of CCL20 production, up regulation of C-C motif chemokine 20 production, up regulation of CCL-20 production, up regulation of CCL20 production, up regulation of chemokine (C-C motif) ligand 20 production, up-regulation of C-C motif chemokine 20 production, up-regulation of CCL-20 production, up-regulation of CCL20 production, up-regulation of chemokine (C-C motif) ligand 20 production, upregulation of C-C motif chemokine 20 production, upregulation of CCL-20 production, upregulation of CCL20 production, upregulation of chemokine (C-C motif) ligand 20 production, activation of C-C motif chemokine 20 production, activation of CCL-20 production, activation of CCL20 production, activation of chemokine (C-C motif) ligand 20 production References: PMID:20054338 Sources: GOC:TermGenie, GOC:krc, GO_REF:0000058 Relationships: is_a GO:0032722; is a type of GO:1903884; positively regulates GO:0036392 Definition: Any process that activates or increases the frequency, rate or extent of chemokine (C-C motif) ligand 20 production.